{
  "term_id": "GO:0090263",
  "term_label": "positive regulation of canonical Wnt signaling pathway",
  "gene_symbol": "NRBP1",
  "gene_name": "Nuclear receptor-binding protein",
  "gene": "UniProtKB:Q9UHY1"
}